{
  "gene_symbol": "SPECC1L",
  "term_id": "UNKNOWN:0001",
  "term_label": "Unknown molecular function",
  "gene_name": "Cytospin-A",
  "gene": "UniProtKB:Q69YQ0"
}